{
  "gene_name": "Dicarboxylate carrier SLC25A8",
  "gene": "UniProtKB:P55851",
  "term_label": "response to cold",
  "gene_symbol": "UCP2",
  "term_id": "GO:0009409"
}